{
  "term_id": "GO:0005874",
  "gene_name": "Microtubule-associated protein 1A",
  "gene": "UniProtKB:P78559",
  "term_label": "microtubule",
  "gene_symbol": "MAP1A"
}